{
  "gene_symbol": "PWWP2B",
  "term_id": "UNKNOWN:0002",
  "gene": "UniProtKB:Q6NUJ5",
  "term_label": "Unknown biological process",
  "gene_name": "PWWP domain-containing protein 2B"
}